positive regulation of acylglycerol transport [GO:1901508] (BP) Subtypes: GO:1905885 Also known as: positive regulation of glyceride transport, up regulation of acylglycerol transport, up regulation of glyceride transport, up-regulation of acylglycerol transport, up-regulation of glyceride transport, upregulation of acylglycerol transport, upregulation of glyceride transport, activation of acylglycerol transport, activation of glyceride transport Relationships: is_a positive regulation of lipid transport [GO:0032370]; is a type of regulation of acylglycerol transport [GO:1901506]; positively regulates GO:0034196 Sources: GOC:TermGenie, GOC:sart Definition: Any process that activates or increases the frequency, rate or extent of acylglycerol transport.